positive regulation of protein localization to presynapse [GO:1905386] (biological process) Definition: Any process that activates or increases the frequency, rate or extent of protein localization to presynapse. References: PMID:24449494 Sources: GOC:PARL, GOC:TermGenie, GOC:bf, GO_REF:0000058 Also known as: positive regulation of protein localisation in presynapse, positive regulation of protein localisation to presynapse, positive regulation of protein localization in presynapse, positive regulation of recruitment of presynaptic proteins, up regulation of protein localisation in presynapse, up regulation of protein localisation to presynapse, up regulation of protein localization in presynapse, up regulation of protein localization to presynapse, up regulation of recruitment of presynaptic proteins, up-regulation of protein localisation in presynapse, up-regulation of protein localisation to presynapse, up-regulation of protein localization in presynapse, up-regulation of protein localization to presynapse, up-regulation of recruitment of presynaptic proteins, upregulation of protein localisation in presynapse, upregulation of protein localisation to presynapse, upregulation of protein localization in presynapse, upregulation of protein localization to presynapse, upregulation of recruitment of presynaptic proteins, activation of protein localisation in presynapse, activation of protein localisation to presynapse, activation of protein localization in presynapse, activation of protein localization to presynapse, activation of recruitment of presynaptic proteins Relationships: is a type of positive regulation of protein localization to synapse [GO:1902474]; is a type of regulation of protein localization to presynapse [GO:1905384]; positively regulates GO:1905383